regulation of lateral mesodermal cell fate specification [GO:0048378] (biological process) Relationships: is a type of regulation of mesodermal cell fate specification [GO:0042661]; regulates GO:0048377 Also known as: regulation of lateral plate mesodermal cell fate specification Sources: GOC:jid Definition: Any process that modulates the frequency, rate or extent of lateral mesoderm cell fate specification. Subtypes: GO:0048379, negative regulation of lateral mesodermal cell fate specification [GO:0048380]